{
  "gene": "UniProtKB:Q12951",
  "term_label": "DNA-binding transcription factor activity, RNA polymerase II-specific",
  "gene_symbol": "FOXI1",
  "gene_name": "Forkhead box protein I1",
  "term_id": "GO:0000981"
}